negative regulation of signaling receptor activity [GO:2000272] (biological process) Relationships: is a type of regulation of signaling receptor activity [GO:0010469]; is_a negative regulation of molecular function [GO:0044092]; negatively regulates GO:0038023 Also known as: negative regulation of receptor activity, negative regulation of signalling receptor activity Subtypes: GO:0007175, cross-receptor inhibition within G protein-coupled receptor heterodimer [GO:0038041], negative regulation of corticotropin-releasing hormone receptor activity [GO:1900011], negative regulation of NMDA glutamate receptor activity [GO:1904782] Definition: Any process that stops, prevents or reduces the frequency, rate or extent of a signaling receptor activity. Sources: GOC:obol